cellular response to interleukin-17 [GO:0097398] (biological process) Definition: Any process that results in a change in state or activity of a cell (in terms of movement, secretion, enzyme production, gene expression, etc.) as a result of an interleukin-17 stimulus. Also known as: cellular response to IL-17 Relationships: is a type of cellular response to cytokine stimulus [GO:0071345]; is a type of response to interleukin-17 [GO:0097396] Sources: GOC:pr